negative regulation of behavior [GO:0048521] (biological process) Also known as: down regulation of behavior, down-regulation of behavior, downregulation of behavior, inhibition of behavior Sources: GOC:jid, GOC:pr Subtypes: negative regulation of host-seeking behavior [GO:0032539], negative regulation of circadian sleep/wake cycle, sleep [GO:0042321], negative regulation of locomotion involved in locomotory behavior [GO:0090327], GO:1901045, negative regulation of male mating behavior [GO:1902436], GO:1903369, negative regulation of locomotor rhythm [GO:1904060], GO:1904326, GO:1905791, GO:2000252, negative regulation of behavioral fear response [GO:2000986] Relationships: is a type of regulation of behavior [GO:0050795]; is a type of GO:0051241; negatively regulates behavior [GO:0007610] Definition: Any process that stops, prevents, or reduces the frequency, rate or extent of behavior, the internally coordinated responses (actions or inactions) of whole living organisms (individuals or groups) to internal or external stimuli.